{
  "gene": "UniProtKB:Q8NEN0",
  "gene_symbol": "ARMC2",
  "gene_name": "Armadillo repeat-containing protein 2",
  "term_id": "GO:0044782",
  "term_label": "cilium organization"
}